{
  "gene_name": "Rap guanine nucleotide exchange factor 2",
  "term_label": "guanyl-nucleotide exchange factor activity",
  "term_id": "GO:0005085",
  "gene": "UniProtKB:Q9Y4G8",
  "gene_symbol": "RAPGEF2"
}